{
  "term_id": "GO:0043014",
  "gene_symbol": "TBCE",
  "gene": "UniProtKB:Q15813",
  "term_label": "alpha-tubulin binding",
  "gene_name": "Tubulin-specific chaperone E"
}